{
  "gene": "UniProtKB:Q8WXI9",
  "gene_symbol": "GATAD2B",
  "term_id": "GO:0016581",
  "gene_name": "Transcriptional repressor p66-beta",
  "term_label": "NuRD complex"
}